nephron tubule formation [GO:0072079] (biological process) Relationships: is a type of GO:0001838; is part of nephron tubule morphogenesis [GO:0072078] Sources: GOC:mtg_kidney_jan10 Subtypes: pronephric nephron tubule formation [GO:0039006], mesonephric tubule formation [GO:0072172], metanephric nephron tubule formation [GO:0072289] Definition: The developmental process pertaining to the initial formation of a nephron tubule from unspecified parts. A nephron tubule is an epithelial tube that is part of the nephron, the functional part of the kidney.